{
  "gene_symbol": "PLIN3",
  "gene": "UniProtKB:O60664",
  "term_label": "lipid droplet",
  "term_id": "GO:0005811",
  "gene_name": "Perilipin-3"
}